{
  "gene": "UniProtKB:P20848",
  "gene_symbol": "SERPINA2",
  "term_id": "GO:0005615",
  "term_label": "extracellular space",
  "gene_name": "Alpha-1-antitrypsin-related protein"
}